conversion of aspartyl-tRNA to asparaginyl-tRNA [GO:0043688] (biological process) References: PMID:9789001 Sources: GOC:jsg Relationships: is a type of charged-tRNA amino acid modification [GO:0019988] Definition: The modification process that results in the conversion of aspartate charged on a tRNA(Asn) to asparaginyl-tRNA. Note: Note that this process has been observed in some archaeal and bacterial species.